{
  "term_id": "UNKNOWN:0002",
  "gene": "UniProtKB:Q6XPR3",
  "gene_name": "Repetin",
  "gene_symbol": "RPTN",
  "term_label": "Unknown biological process"
}